regulation of stem cell population maintenance [GO:2000036] (biological process) Also known as: regulation of maintenance of pluripotency Relationships: is a type of regulation of developmental process [GO:0050793]; is a type of GO:0051239; regulates GO:0019827 Sources: GOC:obol Subtypes: negative regulation of stem cell population maintenance [GO:1902455], GO:1902459, regulation of somatic stem cell population maintenance [GO:1904672] Definition: Any process that modulates the frequency, rate or extent of stem cell population maintenance.